{
  "gene": "UniProtKB:Q96SN7",
  "gene_symbol": "ORAI2",
  "term_label": "store-operated calcium entry",
  "term_id": "GO:0002115",
  "gene_name": "Protein orai-2"
}